{
  "gene_symbol": "NPTXR",
  "gene_name": "Neuronal pentraxin receptor",
  "gene": "UniProtKB:O95502",
  "term_label": "Unknown cellular component",
  "term_id": "UNKNOWN:0003"
}